{
  "gene": "UniProtKB:Q7L3B6",
  "gene_name": "Hsp90 co-chaperone Cdc37-like 1",
  "term_id": "GO:0005737",
  "gene_symbol": "CDC37L1",
  "term_label": "cytoplasm"
}